{
  "term_id": "GO:0099184",
  "gene_symbol": "NEFH",
  "term_label": "structural constituent of postsynaptic intermediate filament cytoskeleton",
  "gene": "UniProtKB:P12036",
  "gene_name": "Neurofilament heavy polypeptide"
}